{
  "gene_symbol": "SESN3",
  "term_id": "GO:0016239",
  "gene_name": "Sestrin-3",
  "term_label": "positive regulation of macroautophagy",
  "gene": "UniProtKB:P58005"
}